{
  "term_id": "GO:0045494",
  "term_label": "photoreceptor cell maintenance",
  "gene": "UniProtKB:P56715",
  "gene_name": "Oxygen-regulated protein 1",
  "gene_symbol": "RP1"
}